{
  "gene": "UniProtKB:P0CJ88",
  "term_id": "GO:0000977",
  "gene_symbol": "DUX4L5",
  "gene_name": "Double homeobox protein 4-like protein 5",
  "term_label": "RNA polymerase II transcription regulatory region sequence-specific DNA binding"
}